{
  "gene_symbol": "CSNK1A1L",
  "gene_name": "Casein kinase I isoform alpha-like",
  "term_label": "signal transduction",
  "gene": "UniProtKB:Q8N752",
  "term_id": "GO:0007165"
}